{
  "gene_symbol": "CPNE1",
  "gene_name": "Copine-1",
  "term_id": "GO:0005544",
  "term_label": "calcium-dependent phospholipid binding",
  "gene": "UniProtKB:Q99829"
}